inosine biosynthetic process [GO:0046103] (biological process) Definition: The chemical reactions and pathways resulting in the formation of inosine, hypoxanthine riboside, a nucleoside found free but not in combination in nucleic acids except in the anticodons of some tRNAs. Relationships: is a type of GO:0046102; is a type of GO:0046129 Also known as: inosine anabolism, inosine biosynthesis, inosine formation, inosine synthesis Subtypes: GO:0006190 Sources: GOC:go_curators